{
  "gene": "UniProtKB:Q9ULH1",
  "term_id": "GO:0032588",
  "gene_name": "Arf-GAP with SH3 domain, ANK repeat and PH domain-containing protein 1",
  "term_label": "trans-Golgi network membrane",
  "gene_symbol": "ASAP1"
}